phosphotransferase activity, for other substituted phosphate groups [GO:0016780] (molecular function) Definition: Catalysis of the transfer of a substituted phosphate group, other than diphosphate or nucleotidyl residues, from one compound (donor) to a another (acceptor). Relationships: is a type of transferase activity, transferring phosphorus-containing groups [GO:0016772] Sources: EC:2.7.8.- Subtypes: ceramide phosphoethanolamine synthase activity [GO:0002950], UDP-N-acetylglucosamine-dolichyl-phosphate N-acetylglucosaminephosphotransferase activity [GO:0003975], GO:0003976, GO:0008807, GO:0008818, holo-[acyl-carrier-protein] synthase activity [GO:0008897], phosphatidylglycerol-membrane-oligosaccharide glycerophosphotransferase activity [GO:0008960], GO:0008963, GO:0017169, GDP-mannose:serine-protein mannose-1-phosphotransferase activity [GO:0018422], GO:0030572, sphingomyelin synthase activity [GO:0033188], UDP-N-acetylglucosamine-undecaprenyl-phosphate N-acetylglucosaminephosphotransferase activity [GO:0036380], archaetidylserine synthase activity [GO:0043761], phosphatidylethanolamine:Kdo2-lipid A phosphoethanolamine transferase activity [GO:0043838], triphosphoribosyl-dephospho-CoA synthase activity [GO:0046917], GO:0047354, CDP-glycerol glycerophosphotransferase activity [GO:0047355], GO:0047356, UDP-galactose-UDP-N-acetylglucosamine galactose phosphotransferase activity [GO:0047357], UDP-glucose-glycoprotein glucose phosphotransferase activity [GO:0047358], 1-alkenyl-2-acylglycerol choline phosphotransferase activity [GO:0047359], undecaprenyl-phosphate galactose phosphotransferase activity [GO:0047360], phosphomannan mannosephosphotransferase activity [GO:0047361], ceramide cholinephosphotransferase activity [GO:0047493], serine-phosphoethanolamine synthase activity [GO:0047494], GO:0047495, phosphatidylcholine synthase activity [GO:0050520], adenosylcobinamide-GDP ribazoletransferase activity [GO:0051073], mannose-ethanolamine phosphotransferase activity [GO:0051377], UDP-N-acetylmuramoyl-L-alanyl-D-glutamyl-meso-2,6-diaminopimelyl-D-alanyl-D-alanine:undecaprenyl-phosphate transferase activity [GO:0051992], alpha-D-ribose 1-methylphosphonate 5-triphosphate synthase activity [GO:0061693], GO:0089702, GO:0102249, N,N'-diacetylbacilliosaminyl-1-phosphate transferase activity [GO:0102334], L-serine-phosphatidylethanolamine phosphatidyltransferase activity [GO:0106245], L-serine-phosphatidylcholine phosphatidyltransferase activity [GO:0106258]